{
  "gene": "UniProtKB:O00264",
  "term_id": "GO:0016020",
  "gene_name": "Membrane-associated progesterone receptor component 1",
  "gene_symbol": "PGRMC1",
  "term_label": "membrane"
}